{
  "term_id": "UNKNOWN:0001",
  "gene_symbol": "TNFRSF13B",
  "term_label": "Unknown molecular function",
  "gene": "UniProtKB:O14836",
  "gene_name": "Tumor necrosis factor receptor superfamily member 13B"
}